{
  "gene_name": "Ubiquinone biosynthesis O-methyltransferase, mitochondrial",
  "term_label": "ubiquinone biosynthetic process",
  "term_id": "GO:0006744",
  "gene_symbol": "COQ3",
  "gene": "UniProtKB:Q9NZJ6"
}